{
  "gene_symbol": "AMFR",
  "gene_name": "E3 ubiquitin-protein ligase AMFR",
  "gene": "UniProtKB:Q9UKV5",
  "term_id": "GO:0000151",
  "term_label": "ubiquitin ligase complex"
}